{
  "term_id": "UNKNOWN:0001",
  "term_label": "Unknown molecular function",
  "gene_name": "Protein PALS1",
  "gene_symbol": "PALS1",
  "gene": "UniProtKB:Q8N3R9"
}